{
  "gene_name": "Natural cytotoxicity triggering receptor 2",
  "gene_symbol": "NCR2",
  "term_label": "signaling receptor activity",
  "gene": "UniProtKB:O95944",
  "term_id": "GO:0038023"
}